double-strand break repair via break-induced replication [GO:0000727] (biological process) Regulation: regulated by regulation of double-strand break repair via break-induced replication [GO:1901591]; negatively regulated by negative regulation of double-strand break repair via break-induced replication [GO:1901592] Definition: The error-free repair of a double-strand break in DNA in which the centromere-proximal end of a broken chromosome searches for a homologous region in an intact chromosome. DNA synthesis initiates from the 3' end of the invading DNA strand, using the intact chromosome as the template, and progresses to the end of the chromosome. Relationships: is a type of double-strand break repair via homologous recombination [GO:0000724] References: PMID:10357855 Sources: GOC:elh